{
  "term_id": "GO:0009898",
  "gene_symbol": "RGS20",
  "term_label": "cytoplasmic side of plasma membrane",
  "gene_name": "Regulator of G-protein signaling 20",
  "gene": "UniProtKB:O76081"
}